{
  "term_id": "GO:0005911",
  "gene": "UniProtKB:Q5EBL8",
  "gene_symbol": "PDZD11",
  "gene_name": "PDZ domain-containing protein 11",
  "term_label": "cell-cell junction"
}